{
  "term_id": "GO:0050911",
  "gene_name": "Olfactory receptor 2L3",
  "gene": "UniProtKB:Q8NG85",
  "gene_symbol": "OR2L3",
  "term_label": "detection of chemical stimulus involved in sensory perception of smell"
}